{
  "term_id": "GO:0015143",
  "gene_symbol": "SLC17A3",
  "gene_name": "Sodium-dependent phosphate transport protein 4",
  "gene": "UniProtKB:O00476",
  "term_label": "urate transmembrane transporter activity"
}